sucrose catabolic process to fructose-6-phosphate and glucose-6-phosphate [GO:0036008] (biological process) Definition: The chemical reactions and pathways resulting in the breakdown of sucrose, which proceeds by phosphorylation of sucrose to form sucrose-6-phosphate. The subsequent actions of a hydrolase and a fructokinase generate fructose-6-phosphate and glucose-6-phosphate. Relationships: is a type of GO:0005987; is a type of GO:0006002; is a type of glucose 6-phosphate metabolic process [GO:0051156]; has part GO:0008865; has part protein-N(PI)-phosphohistidine-sucrose phosphotransferase system transporter activity [GO:0022878]; has part sucrose-phosphate phosphatase activity [GO:0050307] Sources: GOC:bf, GOC:dgf, MetaCyc:SUCUTIL-PWY